melibiose binding [GO:1903777] (molecular function) Definition: Binding to melibiose. References: PMID:11471732 Sources: GOC:TermGenie, GOC:mr, GO_REF:0000067 Relationships: is a type of disaccharide binding [GO:0048030]